{
  "gene": "UniProtKB:Q9NVV5",
  "term_label": "endomembrane system",
  "gene_name": "Androgen-induced gene 1 protein",
  "term_id": "GO:0012505",
  "gene_symbol": "AIG1"
}